{
  "gene": "UniProtKB:Q9Y2P5",
  "gene_symbol": "SLC27A5",
  "term_id": "GO:0005789",
  "gene_name": "Long-chain fatty acid transport protein 5",
  "term_label": "endoplasmic reticulum membrane"
}